{
  "term_id": "GO:0008289",
  "term_label": "lipid binding",
  "gene_name": "Apolipoprotein L6",
  "gene_symbol": "APOL6",
  "gene": "UniProtKB:Q9BWW8"
}